heterophilic cell-cell adhesion [GO:0007157] (biological process) Relationships: is a type of cell-cell adhesion [GO:0098609] Also known as: agglutination Sources: ISBN:0198506732 Definition: The attachment of an adhesion molecule in one cell to a nonidentical adhesion molecule in an adjacent cell.